{
  "term_id": "GO:0051726",
  "gene_symbol": "JUN",
  "gene_name": "Transcription factor Jun",
  "term_label": "regulation of cell cycle",
  "gene": "UniProtKB:P05412"
}